{
  "gene_name": "Low-density lipoprotein receptor class A domain-containing protein 2",
  "gene_symbol": "LDLRAD2",
  "term_id": "UNKNOWN:0003",
  "term_label": "Unknown cellular component",
  "gene": "UniProtKB:Q5SZI1"
}